{
  "term_label": "adenosine to inosine editing",
  "gene_name": "Double-stranded RNA-specific adenosine deaminase",
  "term_id": "GO:0006382",
  "gene_symbol": "ADAR",
  "gene": "UniProtKB:P55265"
}